{
  "term_label": "RNA polymerase II cis-regulatory region sequence-specific DNA binding",
  "gene_symbol": "ZNF774",
  "gene": "UniProtKB:Q6NX45",
  "gene_name": "Zinc finger protein 774",
  "term_id": "GO:0000978"
}